chromatoid body [GO:0033391] (cellular component) Relationships: is a type of cytoplasmic ribonucleoprotein granule [GO:0036464] Definition: A ribonucleoprotein complex found in the cytoplasm of male germ cells, composed of exceedingly thin filaments that are consolidated into a compact mass or into dense strands of varying thickness that branch to form an irregular network. Contains mRNAs, miRNAs, and protein components involved in miRNA processing (such as Argonaute proteins and the endonuclease Dicer) and in RNA decay (such as the decapping enzyme DCP1a and GW182). References: PMID:17183363